{
  "gene": "UniProtKB:Q16527",
  "term_label": "muscle tissue development",
  "gene_name": "Cysteine and glycine-rich protein 2",
  "gene_symbol": "CSRP2",
  "term_id": "GO:0060537"
}